activated CD4-positive, alpha-beta T cell proliferation [GO:0035741] (biological process) Definition: The expansion of an activated CD4-positive, alpha-beta T cell population by cell division. Relationships: is a type of CD4-positive, alpha-beta T cell proliferation [GO:0035739] Sources: CL:0000896, GOC:BHF